{
  "gene": "UniProtKB:P84243",
  "term_id": "GO:0000776",
  "term_label": "kinetochore",
  "gene_name": "Histone H3.3",
  "gene_symbol": "H3-3B"
}